{
  "gene_symbol": "BBC3",
  "gene_name": "Bcl-2-binding component 3, isoforms 3_4",
  "term_id": "GO:0001836",
  "gene": "UniProtKB:Q96PG8",
  "term_label": "release of cytochrome c from mitochondria"
}